interleukin-12-mediated signaling pathway [GO:0035722] (biological process) Definition: The series of molecular signals initiated by interleukin-12 binding to its receptor on the surface of a target cell, and ending with the regulation of a downstream cellular process, e.g. transcription. Relationships: is a type of cytokine-mediated signaling pathway [GO:0019221]; is part of cellular response to interleukin-12 [GO:0071349] Also known as: IL-12-mediated signaling pathway, interleukin-12-mediated signalling pathway Sources: GOC:BHF, GOC:signaling